{
  "gene": "UniProtKB:A6NER0",
  "term_id": "GO:0005096",
  "term_label": "GTPase activator activity",
  "gene_name": "TBC1 domain family member 3F",
  "gene_symbol": "TBC1D3F"
}